{
  "gene": "UniProtKB:Q9NSA2",
  "gene_name": "Potassium voltage-gated channel subfamily D member 1",
  "term_id": "GO:0008076",
  "gene_symbol": "KCND1",
  "term_label": "voltage-gated potassium channel complex"
}